gibberellic acid transmembrane transport [GO:1905200] (BP) Relationships: is a type of terpenoid transport [GO:0046865]; is a type of carboxylic acid transmembrane transport [GO:1905039] References: PMID:27139299 Sources: GOC:TermGenie, GO_REF:0000069 Definition: The directed movement of gibberellic acid across a membrane.